{
  "gene": "UniProtKB:Q8NBJ5",
  "gene_symbol": "COLGALT1",
  "term_label": "Unknown cellular component",
  "gene_name": "Procollagen galactosyltransferase 1",
  "term_id": "UNKNOWN:0003"
}